positive regulation of thymocyte apoptotic process [GO:0070245] (biological process) Relationships: is a type of GO:0070234; is a type of GO:0070243; positively regulates thymocyte apoptotic process [GO:0070242] Note: Note that a thymocyte is an immature T cell located in the thymus (CL:0000893). Also known as: up regulation of thymocyte apoptosis, up-regulation of thymocyte apoptosis, upregulation of thymocyte apoptosis, activation of thymocyte apoptosis, positive regulation of thymocyte apoptosis, stimulation of thymocyte apoptosis, positive regulation of immature T cell apoptosis Definition: Any process that activates or increases the frequency, rate or extent of thymocyte death by apoptotic process. Sources: GOC:add, GOC:mtg_apoptosis, ISBN:0781765196